{
  "gene": "UniProtKB:Q02161",
  "term_id": "GO:0008519",
  "term_label": "ammonium channel activity",
  "gene_symbol": "RHD",
  "gene_name": "Blood group Rh(D) polypeptide"
}